{
  "gene_symbol": "IL17F",
  "gene": "UniProtKB:Q96PD4",
  "term_label": "Unknown cellular component",
  "term_id": "UNKNOWN:0003",
  "gene_name": "Interleukin-17F"
}